{
  "gene": "UniProtKB:Q92796",
  "term_label": "cell-cell adhesion",
  "term_id": "GO:0098609",
  "gene_symbol": "DLG3",
  "gene_name": "Disks large homolog 3"
}